negative regulation of hydrogen peroxide-induced neuron intrinsic apoptotic signaling pathway [GO:1903384] (biological process) Definition: Any process that stops, prevents or reduces the frequency, rate or extent of a hydrogen peroxide-induced neuron intrinsic apoptotic signaling pathway. Also known as: down regulation of H2O2-induced neuron intrinsic apoptotic signaling pathway, down regulation of neuron intrinsic apoptotic signaling pathway in response to H2O2, down regulation of neuron intrinsic apoptotic signaling pathway in response to hydrogen peroxide, down-regulation of H2O2-induced neuron intrinsic apoptotic signaling pathway, down-regulation of neuron intrinsic apoptotic signaling pathway in response to H2O2, down-regulation of neuron intrinsic apoptotic signaling pathway in response to hydrogen peroxide, downregulation of H2O2-induced neuron intrinsic apoptotic signaling pathway, downregulation of neuron intrinsic apoptotic signaling pathway in response to H2O2, downregulation of neuron intrinsic apoptotic signaling pathway in response to hydrogen peroxide, negative regulation of H2O2-induced neuron intrinsic apoptotic signaling pathway, negative regulation of neuron intrinsic apoptotic signaling pathway in response to H2O2, negative regulation of neuron intrinsic apoptotic signaling pathway in response to hydrogen peroxide, inhibition of H2O2-induced neuron intrinsic apoptotic signaling pathway, inhibition of neuron intrinsic apoptotic signaling pathway in response to H2O2, inhibition of neuron intrinsic apoptotic signaling pathway in response to hydrogen peroxide, down regulation of neuron apoptosis in response to hydrogen peroxide, down-regulation of neuron apoptosis in response to hydrogen peroxide, downregulation of neuron apoptosis in response to hydrogen peroxide, inhibition of neuron apoptosis in response to hydrogen peroxide, negative regulation of neuron apoptosis in response to hydrogen peroxide, protection against H2O2-induced neuron apoptosis, protection against hydrogen peroxide-induced neuron apoptosis References: PMID:23261939 Sources: GOC:PARL, GOC:TermGenie, GOC:bf, GO_REF:0000058 Relationships: is a type of negative regulation of oxidative stress-induced neuron intrinsic apoptotic signaling pathway [GO:1903377]; is a type of regulation of hydrogen peroxide-induced neuron intrinsic apoptotic signaling pathway [GO:1903383]; is a type of negative regulation of intrinsic apoptotic signaling pathway in response to hydrogen peroxide [GO:1903751]; RO_0002212 neuron intrinsic apoptotic signaling pathway in response to hydrogen peroxide [GO:0036482]